N-acetylhexosamine 1-dehydrogenase activity [GO:0050120] (molecular function) Sources: EC:1.1.1.240, RHEA:23144 Definition: Catalysis of the reaction: N-acetyl-D-glucosamine + H2O + NAD+ = N-acetyl-D-glucosaminate + 2 H+ + NADH. Relationships: is a type of oxidoreductase activity, acting on the CH-OH group of donors, NAD or NADP as acceptor [GO:0016616] Also known as: N-acetyl-D-hexosamine dehydrogenase activity, N-acetyl-D-hexosamine:NAD+ 1-oxidoreductase activity, N-acetylhexosamine dehydrogenase activity